{
  "gene_symbol": "UXT",
  "term_id": "GO:0003714",
  "gene": "UniProtKB:Q9UBK9",
  "gene_name": "Protein UXT",
  "term_label": "transcription corepressor activity"
}